{
  "gene_symbol": "CFP",
  "gene_name": "Properdin",
  "term_label": "Unknown biological process",
  "gene": "UniProtKB:P27918",
  "term_id": "UNKNOWN:0002"
}